{
  "gene": "UniProtKB:O15540",
  "gene_name": "Fatty acid-binding protein, brain",
  "term_id": "GO:0015908",
  "term_label": "fatty acid transport",
  "gene_symbol": "FABP7"
}